{
  "term_id": "UNKNOWN:0001",
  "gene": "UniProtKB:Q8IUI4",
  "gene_name": "Putative protein SNX29P2",
  "gene_symbol": "SNX29P2",
  "term_label": "Unknown molecular function"
}